{
  "gene_symbol": "FGF2",
  "gene_name": "Fibroblast growth factor 2",
  "term_id": "GO:0008083",
  "term_label": "growth factor activity",
  "gene": "UniProtKB:P09038"
}